{
  "gene": "UniProtKB:Q8TD26",
  "gene_name": "Chromodomain-helicase-DNA-binding protein 6",
  "gene_symbol": "CHD6",
  "term_label": "chromatin binding",
  "term_id": "GO:0003682"
}